positive regulation of motor neuron apoptotic process [GO:2000673] (biological process) Sources: GOC:mtg_apoptosis, GOC:obol Definition: Any process that activates or increases the frequency, rate or extent of motor neuron apoptotic process. Relationships: is a type of positive regulation of neuron apoptotic process [GO:0043525]; is a type of GO:2000671; positively regulates GO:0097049 Also known as: positive regulation of motoneuron apoptosis, positive regulation of motor neuron apoptosis